leukotriene signaling pathway [GO:0061737] (biological process) Relationships: is a type of G protein-coupled receptor signaling pathway [GO:0007186] Definition: A G protein-coupled receptor signaling pathway initiated by leukotriene binding to its receptor on the surface of a target cell, and ending with the regulation of a downstream cellular process. References: PMID:21771892 Sources: GOC:dph